{
  "gene_name": "Protein FAM83H",
  "term_id": "GO:0019901",
  "gene": "UniProtKB:Q6ZRV2",
  "term_label": "protein kinase binding",
  "gene_symbol": "FAM83H"
}